mesenchymal-endodermal cell signaling involved in lung induction [GO:0060493] (BP) Also known as: mesenchymal-endodermal cell signalling involved in lung induction Sources: GOC:dph, GOC:mtg_lung Definition: Any process that mediates the transfer of information from a mesenchymal cell to an endodermal cell in the foregut and contributes to the formation of the lung bud. Relationships: is a type of GO:0060494; is a type of mesenchymal-epithelial cell signaling involved in lung development [GO:0060496]; is a type of mesenchymal-endodermal cell signaling [GO:0060497]; is part of GO:0060492